arylsulfate sulfotransferase activity [GO:0047686] (molecular function) Sources: EC:2.8.2.22, MetaCyc:ARYLSULFATE-SULFOTRANSFERASE-RXN Relationships: is a type of sulfotransferase activity [GO:0008146] Also known as: arylsulfotransferase, arylsulphate sulphotransferase activity, ASST, arylsulfate-phenol sulfotransferase activity, arylsulfate:phenol sulfotransferase activity Definition: Catalysis of the reaction: an aryl sulfate + a phenol = a phenol + an aryl sulfate.